{
  "gene": "UniProtKB:P02792",
  "gene_symbol": "FTL",
  "term_label": "ferric iron binding",
  "term_id": "GO:0008199",
  "gene_name": "Ferritin light chain"
}